{
  "term_id": "UNKNOWN:0002",
  "term_label": "Unknown biological process",
  "gene": "UniProtKB:Q8NH53",
  "gene_symbol": "OR52N1",
  "gene_name": "Olfactory receptor 52N1"
}